{
  "gene": "UniProtKB:P27540",
  "gene_name": "Aryl hydrocarbon receptor nuclear translocator",
  "term_id": "GO:0006357",
  "gene_symbol": "ARNT",
  "term_label": "regulation of transcription by RNA polymerase II"
}